{
  "gene_symbol": "SETD6",
  "term_id": "GO:0016279",
  "gene": "UniProtKB:Q8TBK2",
  "gene_name": "N-lysine methyltransferase SETD6",
  "term_label": "protein-lysine N-methyltransferase activity"
}